{
  "term_label": "Unknown molecular function",
  "gene": "UniProtKB:Q8N6M3",
  "gene_name": "Acyl-coenzyme A diphosphatase FITM2",
  "gene_symbol": "FITM2",
  "term_id": "UNKNOWN:0001"
}